{
  "gene_symbol": "TMEM252",
  "gene": "UniProtKB:Q8N6L7",
  "term_label": "Unknown molecular function",
  "term_id": "UNKNOWN:0001",
  "gene_name": "Transmembrane protein 252"
}